{
  "gene_symbol": "CHKB",
  "term_id": "GO:0006646",
  "gene_name": "Choline_ethanolamine kinase",
  "term_label": "phosphatidylethanolamine biosynthetic process",
  "gene": "UniProtKB:Q9Y259"
}